{
  "gene_name": "Pre-B-cell leukemia transcription factor 4",
  "gene_symbol": "PBX4",
  "gene": "UniProtKB:Q9BYU1",
  "term_id": "GO:0001654",
  "term_label": "eye development"
}